{
  "term_label": "heterochromatin formation",
  "term_id": "GO:0031507",
  "gene_symbol": "H2AC6",
  "gene": "UniProtKB:Q93077",
  "gene_name": "Histone H2A type 1-C"
}